positive regulation of mesonephric glomerulus development [GO:2000089] (biological process) Definition: Any process that activates or increases the frequency, rate or extent of mesonephric glomerulus development. Relationships: is a type of positive regulation of glomerulus development [GO:0090193]; is a type of regulation of mesonephric glomerulus development [GO:2000087]; positively regulates mesonephric glomerulus development [GO:0061224] Sources: GOC:mtg_kidney_jan10